{
  "gene_name": "MICOS complex subunit MIC27",
  "term_label": "cristae formation",
  "term_id": "GO:0042407",
  "gene": "UniProtKB:Q6UXV4",
  "gene_symbol": "APOOL"
}